{
  "gene_symbol": "RHOQ",
  "term_label": "endocytosis",
  "gene": "UniProtKB:P17081",
  "term_id": "GO:0006897",
  "gene_name": "Rho-related GTP-binding protein RhoQ"
}